{
  "term_label": "basement membrane",
  "gene_name": "Laminin subunit alpha-5",
  "gene_symbol": "LAMA5",
  "gene": "UniProtKB:O15230",
  "term_id": "GO:0005604"
}